{
  "term_id": "GO:0051209",
  "gene_name": "1-phosphatidylinositol 4,5-bisphosphate phosphodiesterase epsilon-1",
  "gene": "UniProtKB:Q9P212",
  "gene_symbol": "PLCE1",
  "term_label": "release of sequestered calcium ion into cytosol"
}